{
  "term_id": "GO:0005886",
  "gene": "UniProtKB:O60755",
  "term_label": "plasma membrane",
  "gene_name": "Galanin receptor type 3",
  "gene_symbol": "GALR3"
}